structural constituent of virion [GO:0039660] (molecular function) Definition: The action of a molecule that contributes to the structural integrity of a virion. Sources: GOC:bf, GOC:jl Also known as: viral matrix protein Relationships: is a type of structural molecule activity [GO:0005198]; BFO_0000066 virion component [GO:0044423]